{
  "gene_name": "Small ribosomal subunit protein uS4",
  "term_label": "cytosolic small ribosomal subunit",
  "gene": "UniProtKB:P46781",
  "gene_symbol": "RPS9",
  "term_id": "GO:0022627"
}